{
  "gene_name": "Probable tRNA(His) guanylyltransferase",
  "gene": "UniProtKB:Q9NWX6",
  "term_id": "GO:0008033",
  "gene_symbol": "THG1L",
  "term_label": "tRNA processing"
}